{
  "term_label": "Unknown molecular function",
  "gene": "UniProtKB:Q9NWK9",
  "gene_symbol": "ZNHIT6",
  "gene_name": "Box C_D snoRNA protein 1",
  "term_id": "UNKNOWN:0001"
}